{
  "gene": "UniProtKB:Q9BZC1",
  "gene_symbol": "CELF4",
  "term_id": "GO:0006376",
  "term_label": "mRNA splice site recognition",
  "gene_name": "CUGBP Elav-like family member 4"
}